{
  "term_id": "GO:0048513",
  "gene": "UniProtKB:P0DML3",
  "term_label": "animal organ development",
  "gene_name": "Chorionic somatomammotropin hormone 2",
  "gene_symbol": "CSH2"
}